{
  "gene": "UniProtKB:Q9NRD5",
  "gene_name": "PRKCA-binding protein",
  "term_label": "dendritic spine maintenance",
  "gene_symbol": "PICK1",
  "term_id": "GO:0097062"
}